{
  "gene_symbol": "ERG",
  "gene": "UniProtKB:P11308",
  "term_label": "cell differentiation",
  "gene_name": "Transcriptional regulator ERG",
  "term_id": "GO:0030154"
}